{
  "term_id": "GO:0005737",
  "gene": "UniProtKB:Q8TDR2",
  "gene_name": "Serine_threonine-protein kinase 35",
  "gene_symbol": "STK35",
  "term_label": "cytoplasm"
}